{
  "term_label": "Unknown cellular component",
  "term_id": "UNKNOWN:0003",
  "gene_name": "Putative uncharacterized protein encoded by LINC00322",
  "gene": "UniProtKB:Q6ZN03",
  "gene_symbol": "LINC00322"
}